{
  "gene_symbol": "NUGGC",
  "gene_name": "Nuclear GTPase SLIP-GC",
  "term_label": "GTPase activity",
  "gene": "UniProtKB:Q68CJ6",
  "term_id": "GO:0003924"
}